{
  "term_id": "GO:0042015",
  "term_label": "interleukin-20 binding",
  "gene_name": "Interleukin-20 receptor subunit alpha",
  "gene_symbol": "IL20RA",
  "gene": "UniProtKB:Q9UHF4"
}